positive regulation of plant-type cell wall cellulose catabolic process [GO:2000941] (biological process) Definition: Any process that activates or increases the frequency, rate or extent of plant-type cell wall cellulose catabolic process. Sources: GOC:mengo_curators Also known as: positive regulation of plant-type cell wall polysaccharide breakdown Relationships: is a type of GO:2000939; is a type of positive regulation of cell wall polysaccharide catabolic process [GO:2000968]; positively regulates plant-type cell wall cellulose catabolic process [GO:0044348]